{
  "term_id": "GO:0000978",
  "gene": "UniProtKB:Q76KX8",
  "gene_symbol": "ZNF534",
  "gene_name": "Zinc finger protein 534",
  "term_label": "RNA polymerase II cis-regulatory region sequence-specific DNA binding"
}